{
  "term_id": "GO:0033693",
  "gene_name": "Neurofilament medium polypeptide",
  "gene_symbol": "NEFM",
  "term_label": "neurofilament bundle assembly",
  "gene": "UniProtKB:P07197"
}